ABC-type sulfate transporter activity [GO:0015419] (molecular function) Also known as: sulfate/thiosulfate porter activity, sulfate ABC transporter, ATPase-coupled sulfate transmembrane transporter activity, sulfate transmembrane-transporting ATPase activity, sulfate-transporting ATPase activity, sulphate transporting ATPase activity Sources: RHEA:10192 Definition: Enables the transfer of a solute or solutes from one side of a membrane to the other according to the reaction: ATP + H2O + sulfate(out) = ADP + phosphate + sulfate(in). Relationships: is a type of sulfate transmembrane transporter activity [GO:0015116]; is_a GO:0140359